{
  "gene_name": "Polymeric immunoglobulin receptor",
  "term_id": "GO:0004888",
  "gene": "UniProtKB:P01833",
  "term_label": "transmembrane signaling receptor activity",
  "gene_symbol": "PIGR"
}